{
  "gene_name": "Putative protein KRIP1",
  "gene_symbol": "KLKP1",
  "term_label": "Unknown molecular function",
  "gene": "UniProtKB:Q107X0",
  "term_id": "UNKNOWN:0001"
}